{
  "gene_symbol": "ZNF28",
  "term_id": "GO:0000978",
  "term_label": "RNA polymerase II cis-regulatory region sequence-specific DNA binding",
  "gene": "UniProtKB:P17035",
  "gene_name": "Zinc finger protein 28"
}